cellular response to epidermal growth factor stimulus [GO:0071364] (biological process) Sources: GOC:mah Definition: Any process that results in a change in state or activity of a cell (in terms of movement, secretion, enzyme production, gene expression, etc.) as a result of an epidermal growth factor stimulus. Also known as: cellular response to EGF stimulus Relationships: is a type of response to epidermal growth factor [GO:0070849]; is a type of cellular response to growth factor stimulus [GO:0071363]